{
  "gene_name": "Putative protein FAM90A20P",
  "term_label": "Unknown cellular component",
  "term_id": "UNKNOWN:0003",
  "gene": "UniProtKB:A6NIJ5",
  "gene_symbol": "FAM90A20P"
}